{
  "term_label": "Unknown molecular function",
  "gene": "UniProtKB:Q9BWV1",
  "gene_symbol": "BOC",
  "term_id": "UNKNOWN:0001",
  "gene_name": "Brother of CDO"
}